{
  "gene": "UniProtKB:Q16698",
  "term_id": "GO:0008670",
  "term_label": "2,4-dienoyl-CoA reductase (NADPH) activity",
  "gene_symbol": "DECR1",
  "gene_name": "2,4-dienoyl-CoA reductase [(3E)-enoyl-CoA-producing], mitochondrial"
}